{
  "term_label": "membrane",
  "gene_symbol": "ACTBL2",
  "term_id": "GO:0016020",
  "gene": "UniProtKB:Q562R1",
  "gene_name": "Beta-actin-like protein 2"
}